meiotic DNA double-strand break processing involved in reciprocal meiotic recombination [GO:0010705] (biological process) Sources: GOC:dph, GOC:tb Definition: The cell cycle process in which the 5' to 3' exonucleolytic resection of the DNA at the site of the break to form a 3' single-strand DNA overhang occurs resulting in double strand break formation and repair through a double Holliday junction intermediate. Relationships: is a type of meiotic DNA double-strand break processing [GO:0000706]; is part of reciprocal meiotic recombination [GO:0007131]